{
  "term_label": "Unknown cellular component",
  "gene": "UniProtKB:Q5SR56",
  "gene_symbol": "MFSD14B",
  "gene_name": "Hippocampus abundant transcript-like protein 1",
  "term_id": "UNKNOWN:0003"
}